pH-gated sodium channel activity [GO:0160125] (molecular function) References: PMID:34767445 Definition: A gated channel activity that enables the transmembrane transfer of a sodium ion by a channel that opens in response to a change in pH. Also known as: pH-dependent sodium channel activity, pH-sensitive sodium channel activity Relationships: is a type of ligand-gated sodium channel activity [GO:0015280]; is a type of pH-gated monoatomic ion channel activity [GO:0160128]